{
  "gene_name": "Ephrin type-B receptor 6",
  "term_id": "GO:0030425",
  "gene": "UniProtKB:O15197",
  "gene_symbol": "EPHB6",
  "term_label": "dendrite"
}